{
  "gene_symbol": "EIF2AK4",
  "term_label": "nucleus",
  "gene_name": "eIF-2-alpha kinase GCN2",
  "term_id": "GO:0005634",
  "gene": "UniProtKB:Q9P2K8"
}